filamentous growth of a population of unicellular organisms in response to pH [GO:0036177] (biological process) Subtypes: GO:0036178 Regulation: regulated by regulation of filamentous growth of a population of unicellular organisms in response to pH [GO:1900741]; negatively regulated by negative regulation of filamentous growth of a population of unicellular organisms in response to pH [GO:1900742]; positively regulated by positive regulation of filamentous growth of a population of unicellular organisms in response to pH [GO:1900743] Relationships: is a type of response to pH [GO:0009268]; is a type of filamentous growth of a population of unicellular organisms [GO:0044182] Definition: The process in which a group of unicellular organisms grow in a threadlike, filamentous shape in response to a pH stimulus. pH is a measure of the acidity or basicity of an aqueous solution. Sources: GOC:di, Wikipedia:PH